{
  "gene_symbol": "ACTC1",
  "gene_name": "Actin, alpha cardiac muscle 1",
  "gene": "UniProtKB:P68032",
  "term_label": "heart contraction",
  "term_id": "GO:0060047"
}